{
  "gene_name": "Galectin-9B",
  "term_id": "GO:0005829",
  "gene_symbol": "LGALS9B",
  "gene": "UniProtKB:Q3B8N2",
  "term_label": "cytosol"
}